{
  "gene_symbol": "IFNL4",
  "term_label": "extracellular space",
  "term_id": "GO:0005615",
  "gene_name": "Interferon lambda-4",
  "gene": "UniProtKB:K9M1U5"
}